carboxylic acid transmembrane transporter activity [GO:0046943] (molecular function) Subtypes: sulfur amino acid transmembrane transporter activity [GO:0000099], beta-alanine transmembrane transporter activity [GO:0001761], glutamate-gated receptor activity [GO:0004970], GO:0005297, proline:sodium symporter activity [GO:0005298], creatine transmembrane transporter activity [GO:0005308], dicarboxylic acid transmembrane transporter activity [GO:0005310], tricarboxylate secondary active transmembrane transporter activity [GO:0005371], UDP-glucuronate transmembrane transporter activity [GO:0005461], monocarboxylic acid transmembrane transporter activity [GO:0008028], folic acid transmembrane transporter activity [GO:0008517], L-ascorbate:sodium symporter activity [GO:0008520], allantoate transmembrane transporter activity [GO:0015124], glucuronate transmembrane transporter activity [GO:0015135], tricarboxylic acid transmembrane transporter activity [GO:0015142], GO:0015173, L-amino acid transmembrane transporter activity [GO:0015179], glycine transmembrane transporter activity [GO:0015187], GO:0015229, 5-formyltetrahydrofolate transmembrane transporter activity [GO:0015231], GO:0015233, GO:0015306, lysine:proton symporter activity [GO:0015493], pantothenate:sodium symporter activity [GO:0015498], GO:0015501, hexuronate:monoatomic cation symporter activity [GO:0015539], galacturonate transmembrane transporter activity [GO:0015550], GO:0015556, branched-chain amino acid transmembrane transporter activity [GO:0015658], alanine transmembrane transporter activity [GO:0022858], ATPase-coupled carboxylic acid transmembrane transporter activity [GO:0033284], aldarate transmembrane transporter activity [GO:0042876], aldonate transmembrane transporter activity [GO:0042879], benzoate transmembrane transporter activity [GO:0042925], achromobactin transmembrane transporter activity [GO:0042934], D-amino acid transmembrane transporter activity [GO:0042943], GO:0043858, arginine:agmatine antiporter activity [GO:0043862], lysine:cadaverine antiporter activity [GO:0043872], GO:0051477, GO:1905201 Sources: GOC:ai Relationships: is a type of transmembrane transporter activity [GO:0022857]; is part of carboxylic acid transmembrane transport [GO:1905039] Definition: Enables the transfer of carboxylic acids from one side of a membrane to the other. Carboxylic acids are organic acids containing one or more carboxyl (COOH) groups or anions (COO-).